intraciliary transport [GO:0042073] (BP) Note: Note that we deem cilium and microtubule-based flagellum to be equivalent. Relationships: is_a transport along microtubule [GO:0010970]; is part of GO:0044782; occurs in cilium [GO:0005929] Also known as: intraflagellar transport, intraflagellar transport involved in cilium organization, intraflagellar transport involved in microtubule-based flagellum organisation, IFT References: PMID:17981739, PMID:18180368, PMID:22869374 Sources: GOC:cilia, GOC:kmv Subtypes: intraciliary anterograde transport [GO:0035720], GO:0035721, GO:0035735 Definition: The bidirectional movement of large protein complexes along microtubules within a cilium, mediated by motor proteins.